gap junction channel activity involved in AV node cell-bundle of His cell electrical coupling [GO:0086077] (molecular function) Sources: GOC:BHF, GOC:mtg_cardiac_conduct_nov11 Definition: A wide pore channel activity that enables a direct cytoplasmic connection from an AV node cell to a bundle of His cell. The gap junction passes electrical signals between the cells contributing to cardiac conduction. Relationships: is a type of gap junction channel activity involved in cardiac conduction electrical coupling [GO:0086075]; is part of AV node cell to bundle of His cell communication by electrical coupling [GO:0086053] Also known as: gap junction channel activity involved in atrioventricular node cell-bundle of His cell electrical coupling